regulation of nitrogen utilization [GO:0006808] (biological process) Subtypes: negative regulation of nitrogen utilization [GO:0045847], positive regulation of nitrogen utilization [GO:0045848], nitrogen catabolite regulation of transcription [GO:0090293], GO:2001248 Relationships: is a type of regulation of response to nutrient levels [GO:0032107]; regulates nitrogen utilization [GO:0019740] Definition: Any process that modulates the frequency, rate or extent of nitrogen utilization. Sources: GOC:go_curators